{
  "term_id": "GO:0016308",
  "gene_name": "Phosphatidylinositol 4-phosphate 5-kinase type-1 beta",
  "gene": "UniProtKB:O14986",
  "gene_symbol": "PIP5K1B",
  "term_label": "1-phosphatidylinositol-4-phosphate 5-kinase activity"
}